{
  "gene_name": "Galanin peptides",
  "term_id": "GO:0030141",
  "gene": "UniProtKB:P22466",
  "term_label": "secretory granule",
  "gene_symbol": "GAL"
}